positive regulation of cardiac ventricle formation [GO:1904944] (biological process) References: PMID:23575307 Sources: GOC:BHF, GOC:BHF_miRNA, GOC:TermGenie, GOC:bc, GO_REF:0000058 Relationships: is a type of positive regulation of cardiac chamber formation [GO:1901212]; is a type of regulation of cardiac ventricle formation [GO:1904942]; positively regulates GO:0003211 Definition: Any process that activates or increases the frequency, rate or extent of cardiac ventricle formation. Also known as: up regulation of cardiac ventricle formation, up-regulation of cardiac ventricle formation, upregulation of cardiac ventricle formation, activation of cardiac ventricle formation